{
  "gene": "UniProtKB:Q9HB75",
  "gene_name": "p53-induced death domain-containing protein 1",
  "gene_symbol": "PIDD1",
  "term_label": "apoptotic process",
  "term_id": "GO:0006915"
}